{
  "gene": "UniProtKB:P18085",
  "gene_symbol": "ARF4",
  "term_label": "cytoplasm",
  "gene_name": "ADP-ribosylation factor 4",
  "term_id": "GO:0005737"
}